psychosine sulfotransferase activity [GO:0050226] (molecular function) Definition: Catalysis of the reaction: 3'-phosphoadenosine 5'-phosphosulfate + galactosylsphingosine = adenosine 3',5'-bisphosphate + psychosine sulfate. Also known as: psychosine sulphotransferase activity, 3'-phosphoadenosine 5'-phosphosulfate-psychosine sulphotransferase activity, 3'-phosphoadenylyl-sulfate:galactosylsphingosine sulfotransferase activity, PAPS:psychosine sulphotransferase activity Sources: EC:2.8.2.13, MetaCyc:PSYCHOSINE-SULFOTRANSFERASE-RXN Relationships: is a type of sulfotransferase activity [GO:0008146]